{
  "gene_name": "Transport and Golgi organization protein 6 homolog",
  "term_id": "GO:0009306",
  "term_label": "protein secretion",
  "gene_symbol": "TANGO6",
  "gene": "UniProtKB:Q9C0B7"
}